{
  "term_id": "GO:0005886",
  "term_label": "plasma membrane",
  "gene_symbol": "AVPR2",
  "gene": "UniProtKB:P30518",
  "gene_name": "Vasopressin V2 receptor"
}